{
  "term_label": "Unknown molecular function",
  "term_id": "UNKNOWN:0001",
  "gene_name": "Putative uncharacterized protein encoded by LINC00469",
  "gene": "UniProtKB:Q8N7U9",
  "gene_symbol": "LINC00469"
}